{
  "gene_symbol": "VPS16",
  "gene_name": "Vacuolar protein sorting-associated protein 16 homolog",
  "gene": "UniProtKB:Q9H269",
  "term_label": "actin binding",
  "term_id": "GO:0003779"
}